chloride ion homeostasis [GO:0055064] (biological process) Relationships: is a type of monoatomic anion homeostasis [GO:0055081]; is a type of inorganic ion homeostasis [GO:0098771] Definition: Any process involved in the maintenance of an internal steady state of chloride ions within an organism or cell. Subtypes: intracellular chloride ion homeostasis [GO:0030644] Sources: GOC:jid, GOC:mah